{
  "gene": "UniProtKB:Q2M2I8",
  "gene_symbol": "AAK1",
  "gene_name": "AP2-associated protein kinase 1",
  "term_id": "GO:0098793",
  "term_label": "presynapse"
}